{
  "gene": "UniProtKB:A6NH52",
  "term_label": "Unknown molecular function",
  "term_id": "UNKNOWN:0001",
  "gene_symbol": "TVP23A",
  "gene_name": "Golgi apparatus membrane protein TVP23 homolog A"
}